{
  "gene_name": "Conserved oligomeric Golgi complex subunit 5",
  "term_label": "intra-Golgi vesicle-mediated transport",
  "term_id": "GO:0006891",
  "gene_symbol": "COG5",
  "gene": "UniProtKB:Q9UP83"
}